positive regulation of protein phosphorylation [GO:0001934] (biological process) Definition: Any process that activates or increases the frequency, rate or extent of addition of phosphate groups to amino acids within a protein. Also known as: positive regulation of protein amino acid phosphorylation, up regulation of protein amino acid phosphorylation, up-regulation of protein amino acid phosphorylation, upregulation of protein amino acid phosphorylation, activation of protein amino acid phosphorylation, stimulation of protein amino acid phosphorylation Sources: GOC:hjd Subtypes: positive regulation of peptidyl-threonine phosphorylation [GO:0010800], GO:0031954, positive regulation of peptidyl-serine phosphorylation [GO:0033138], GO:0045860, GO:0050731, positive regulation of I-kappaB phosphorylation [GO:1903721], GO:1904325 Relationships: is a type of regulation of protein phosphorylation [GO:0001932]; is a type of GO:0031401; is_a GO:0042327; positively regulates protein phosphorylation [GO:0006468]